{
  "term_label": "complement activation",
  "gene_symbol": "C2",
  "gene": "UniProtKB:P06681",
  "gene_name": "Complement C2",
  "term_id": "GO:0006956"
}